negative regulation of dense core granule transport [GO:1904810] (biological process) References: PMID:22699897 Sources: GOC:TermGenie, GO_REF:0000058 Also known as: down regulation of dense core granule transport, down regulation of dense core vesicle transport, down-regulation of dense core granule transport, down-regulation of dense core vesicle transport, downregulation of dense core granule transport, downregulation of dense core vesicle transport, negative regulation of dense core vesicle transport, inhibition of dense core granule transport, inhibition of dense core vesicle transport Subtypes: GO:1901952, negative regulation of retrograde dense core granule transport [GO:1901955] Note: cdk-5 in C.elegans (G5ECH7) in PMID:22699897 (inferred from mutant phenotype). Definition: Any process that stops, prevents or reduces the frequency, rate or extent of dense core granule transport. Relationships: is a type of negative regulation of intracellular transport [GO:0032387]; is a type of regulation of dense core granule transport [GO:1904809]; negatively regulates GO:1901950